{
  "term_label": "Unknown cellular component",
  "gene_symbol": "LINC03043",
  "term_id": "UNKNOWN:0003",
  "gene": "UniProtKB:A4D0Y5",
  "gene_name": "Uncharacterized protein encoded by LINC03043"
}